{
  "gene_name": "Transmembrane protein 59",
  "term_label": "lysosome",
  "gene_symbol": "TMEM59",
  "term_id": "GO:0005764",
  "gene": "UniProtKB:Q9BXS4"
}